{
  "term_label": "Unknown biological process",
  "gene_name": "Putative POM121-like protein 1",
  "gene_symbol": "POM121L1P",
  "term_id": "UNKNOWN:0002",
  "gene": "UniProtKB:Q3SYA9"
}